folate transmembrane transport [GO:0098838] (biological process) Relationships: is_a folic acid transport [GO:0015884]; is a type of vitamin transmembrane transport [GO:0035461]; is a type of carboxylic acid transmembrane transport [GO:1905039] Also known as: reduced folate transmembrane transport, folic acid transmembrane transport Definition: The process in which a folic acid, or one of its derivatives (dihydrofolate, tetrahydrofolate, methylene-tetrahydrofolate or methyl-tetrahydrofolate) is transported across a membrane. References: PMID:24745983 Subtypes: folate import across plasma membrane [GO:1904447], folate import into mitochondrion [GO:1904947]